acyl-CoA oxidase activity [GO:0003997] (molecular function) Subtypes: pristanoyl-CoA oxidase activity [GO:0016402], very-long-chain fatty acyl-CoA oxidase activity [GO:0044535], short-chain fatty acyl-CoA oxidase activity [GO:0120522], medium-chain fatty acyl-CoA oxidase activity [GO:0120523], long-chain fatty acyl-CoA oxidase activity [GO:0120524] Definition: Catalysis of the reaction: a 2,3-saturated acyl-CoA + O2 = a (2E)-enoyl-CoA + H2O2. Sources: RHEA:38959 Also known as: acyl coenzyme A oxidase activity, acyl-CoA:oxygen 2-oxidoreductase activity, fatty acyl-CoA oxidase activity, fatty acyl-coenzyme A oxidase activity Relationships: is a type of oxidoreductase activity, acting on the CH-CH group of donors, oxygen as acceptor [GO:0016634]